{
  "gene_symbol": "LPP",
  "gene_name": "Lipoma-preferred partner",
  "term_label": "focal adhesion",
  "gene": "UniProtKB:Q93052",
  "term_id": "GO:0005925"
}